{
  "gene_symbol": "ALX4",
  "term_id": "GO:0006357",
  "term_label": "regulation of transcription by RNA polymerase II",
  "gene_name": "Homeobox protein aristaless-like 4",
  "gene": "UniProtKB:Q9H161"
}